{
  "gene": "UniProtKB:P00747",
  "gene_name": "Plasminogen",
  "term_id": "GO:0004175",
  "term_label": "endopeptidase activity",
  "gene_symbol": "PLG"
}